{
  "term_label": "plasma membrane",
  "term_id": "GO:0005886",
  "gene": "UniProtKB:Q9GZQ6",
  "gene_symbol": "NPFFR1",
  "gene_name": "Neuropeptide FF receptor 1"
}